negative regulation of preblastoderm mitotic cell cycle [GO:0046001] (biological process) Relationships: is a type of regulation of preblastoderm mitotic cell cycle [GO:0007347]; is a type of negative regulation of mitotic cell cycle, embryonic [GO:0045976]; negatively regulates GO:0035185 Sources: GOC:dph, GOC:go_curators, GOC:tb Also known as: down regulation of progression through preblastoderm mitotic cell cycle, down-regulation of progression through preblastoderm mitotic cell cycle, downregulation of progression through preblastoderm mitotic cell cycle, negative regulation of preblastoderm mitotic cell cycle progression, negative regulation of progression through preblastoderm mitotic cell cycle, inhibition of progression through preblastoderm mitotic cell cycle Definition: Any process that stops, prevents or reduces the rate or extent of progression through the preblastoderm mitotic cell cycle.